negative regulation of biological process [GO:0048519] (biological process) Definition: Any process that stops, prevents, or reduces the frequency, rate or extent of a biological process. Biological processes are regulated by many means; examples include the control of gene expression, protein modification or interaction with a protein or substrate molecule. Sources: GOC:jid Also known as: down regulation of biological process, down-regulation of biological process, downregulation of biological process, negative regulation of physiological process, inhibition of biological process Subtypes: negative regulation of immune system process [GO:0002683], negative regulation of signaling [GO:0023057], negative regulation of border follicle cell delamination [GO:0030712], GO:0032848, negative regulation of GTPase activity [GO:0034260], GO:0040013, negative regulation of circadian rhythm [GO:0042754], negative regulation of formation of structure involved in a symbiotic process [GO:0044147], negative regulation of action potential [GO:0045759], GO:0045926, negative regulation of developmental pigmentation [GO:0048086], negative regulation of cellular process [GO:0048523], GO:0048525, GO:0048585, negative regulation of transport [GO:0051051], negative regulation of developmental process [GO:0051093], negative regulation of multicellular organismal process [GO:0051241], negative regulation of fibrinolysis [GO:0051918], negative regulation of post-transcriptional gene silencing [GO:0060149], negative regulation of gene silencing by regulatory ncRNA [GO:0060967], negative regulation of excitatory postsynaptic potential [GO:0090394], negative regulation of kainate selective glutamate receptor signaling pathway [GO:0106427], negative regulation of interphase mitotic telomere clustering [GO:0110066], negative regulation of hemostasis [GO:1900047], negative regulation of long-term synaptic potentiation [GO:1900272], GO:1900453, negative regulation of membrane hyperpolarization [GO:1902631], negative regulation of receptor localization to synapse [GO:1902684], negative regulation of receptor-mediated virion attachment to host cell [GO:1902735], negative regulation of cardiac conduction [GO:1903780], negative regulation of protein localization [GO:1903828], negative regulation of membrane depolarization [GO:1904180], negative regulation of transformation of host cell by virus [GO:1904188], GO:1904537, GO:1904581, negative regulation of telomerase RNA localization to Cajal body [GO:1904873], negative regulation of establishment of RNA localization to telomere [GO:1904911], negative regulation of establishment of protein-containing complex localization to telomere [GO:1904914], GO:1904950, negative regulation of membrane repolarization during cardiac muscle cell action potential [GO:1905032], GO:1905513, GO:1905869, GO:1905953, negative regulation of reproductive process [GO:2000242], negative regulation of entry of bacterium into host cell [GO:2000536] Relationships: is a type of GO:0050789; negatively regulates biological_process [GO:0008150]